response to tacrolimus [GO:1901327] (biological process) Definition: Any process that results in a change in state or activity of a cell or an organism (in terms of movement, secretion, enzyme production, gene expression, etc.) as a result of a tacrolimus stimulus. Subtypes: cellular response to tacrolimus [GO:0072748] Relationships: is a type of response to nitrogen compound [GO:1901698]; is a type of response to oxygen-containing compound [GO:1901700] Sources: GOC:TermGenie Also known as: response to FK506, response to tacrolimus hydrate